{
  "term_label": "acetylcholine receptor signaling pathway",
  "gene_name": "Acetylcholine receptor subunit delta",
  "gene_symbol": "CHRND",
  "term_id": "GO:0095500",
  "gene": "UniProtKB:Q07001"
}